{
  "term_label": "RNA polymerase II cis-regulatory region sequence-specific DNA binding",
  "gene_name": "DNA-binding protein RFX7",
  "gene": "UniProtKB:Q2KHR2",
  "gene_symbol": "RFX7",
  "term_id": "GO:0000978"
}